{
  "gene_symbol": "SUMO3",
  "term_id": "GO:0005634",
  "gene": "UniProtKB:P55854",
  "gene_name": "Small ubiquitin-related modifier 3",
  "term_label": "nucleus"
}